butanediol catabolic process [GO:0034078] (biological process) Also known as: butanediol breakdown, butanediol catabolism, butanediol degradation, butylene glycol catabolic process, butylene glycol catabolism, butanediol utilization Definition: The chemical reactions and pathways resulting in the breakdown of butanediol; the biologically relevant isomer is 2,3-butanediol, CH3CH(OH)CH(OH)CH3. Relationships: is a type of butanediol metabolic process [GO:0034077]; is a type of glycol catabolic process [GO:0042846] Sources: GOC:mah, ISBN:0911910123